{
  "term_label": "cytosol",
  "gene_symbol": "LTN1",
  "gene_name": "E3 ubiquitin-protein ligase listerin",
  "gene": "UniProtKB:O94822",
  "term_id": "GO:0005829"
}